{
  "gene_symbol": "ATG4B",
  "gene_name": "Cysteine protease ATG4B",
  "gene": "UniProtKB:Q9Y4P1",
  "term_id": "GO:0019786",
  "term_label": "protein-phosphatidylethanolamide deconjugating activity"
}